{
  "term_id": "GO:0045109",
  "gene": "UniProtKB:P35900",
  "term_label": "intermediate filament organization",
  "gene_name": "Keratin, type I cytoskeletal 20",
  "gene_symbol": "KRT20"
}